4-hydroxyglutamate transaminase activity [GO:0047578] (molecular function) Definition: Catalysis of the reaction: 4-hydroxy-L-glutamate + 2-oxoglutarate = 4-hydroxy-2-oxoglutarate + L-glutamate. Also known as: 4-hydroxyglutamate aminotransferase activity, 4-hydroxy-L-glutamate:2-oxoglutarate aminotransferase activity Sources: EC:2.6.1.23, MetaCyc:4-HYDROXYGLUTAMATE-AMINOTRANSFERASE-RXN Relationships: is a type of transaminase activity [GO:0008483]